neuromast support cell differentiation [GO:0048889] (biological process) Subtypes: anterior lateral line neuromast support cell differentiation [GO:0048906], posterior lateral line neuromast support cell differentiation [GO:0048927] Sources: ISBN:0125296509 Relationships: is a type of GO:0030154; is part of GO:0048884 Definition: The process in which a relatively unspecialized cell acquires specialized features of a neuromast support cell. Support cells are non-sensory cells of the neuromast that extend between the sensory hair cells from the basement membrane to the apical surface; they are surrounded by mantle cells.